{
  "term_label": "ubiquitin protein ligase activity",
  "gene": "UniProtKB:Q9UK22",
  "gene_symbol": "FBXO2",
  "gene_name": "F-box only protein 2",
  "term_id": "GO:0061630"
}